aminoacyl-tRNA ligase activity [GO:0004812] (molecular function) Also known as: ligase activity, forming aminoacyl-tRNA and related compounds, aminoacyl-tRNA synthetase activity, aminoacyl-tRNA synthetase auxiliary protein activity Note: Note that the bond resulting from this reaction is a carboxylic acid ester bond, linking the alpha carboxyl group of the amino acid to either the 2' or 3' hydroxyl of the 3'- terminal adenyl residue of the tRNA. Relationships: is a type of ligase activity, forming carbon-oxygen bonds [GO:0016875]; is a type of catalytic activity, acting on a tRNA [GO:0140101] Definition: Catalysis of the formation of aminoacyl-tRNA from ATP, amino acid, and tRNA with the release of diphosphate and AMP. Subtypes: alanine-tRNA ligase activity [GO:0004813], arginine-tRNA ligase activity [GO:0004814], aspartate-tRNA ligase activity [GO:0004815], asparagine-tRNA ligase activity [GO:0004816], cysteine-tRNA ligase activity [GO:0004817], glutamate-tRNA ligase activity [GO:0004818], GO:0004819, glycine-tRNA ligase activity [GO:0004820], histidine-tRNA ligase activity [GO:0004821], GO:0004822, leucine-tRNA ligase activity [GO:0004823], GO:0004824, methionine-tRNA ligase activity [GO:0004825], phenylalanine-tRNA ligase activity [GO:0004826], GO:0004827, serine-tRNA ligase activity [GO:0004828], GO:0004829, GO:0004830, tyrosine-tRNA ligase activity [GO:0004831], valine-tRNA ligase activity [GO:0004832], GO:0043767, phosphoserine-tRNA(Cys) ligase activity [GO:0043816], aspartate-tRNA(Asn) ligase activity [GO:0050560], GO:0050561, GO:0098618, GO:0098619 Sources: ISBN:0198506732 Regulation: positively regulated by GO:0140733